{
  "term_id": "UNKNOWN:0001",
  "term_label": "Unknown molecular function",
  "gene_symbol": "PAM16",
  "gene": "UniProtKB:Q9Y3D7",
  "gene_name": "Mitochondrial import inner membrane translocase subunit TIM16"
}